{
  "term_id": "UNKNOWN:0001",
  "gene_symbol": "OOSP4A",
  "gene_name": "Oocyte-secreted protein 4A",
  "term_label": "Unknown molecular function",
  "gene": "UniProtKB:A0A2R8YFL7"
}